{
  "term_label": "spermatid nucleus differentiation",
  "gene": "UniProtKB:P52594",
  "term_id": "GO:0007289",
  "gene_symbol": "AGFG1",
  "gene_name": "Arf-GAP domain and FG repeat-containing protein 1"
}